{
  "gene_name": "5-hydroxytryptamine receptor 6",
  "gene_symbol": "HTR6",
  "gene": "UniProtKB:P50406",
  "term_label": "chemical synaptic transmission",
  "term_id": "GO:0007268"
}